{
  "gene_name": "Nuclear envelope integral membrane protein 1",
  "term_id": "UNKNOWN:0001",
  "term_label": "Unknown molecular function",
  "gene": "UniProtKB:O14524",
  "gene_symbol": "NEMP1"
}